{
  "term_label": "Unknown biological process",
  "gene_name": "Dipeptidyl peptidase 3",
  "term_id": "UNKNOWN:0002",
  "gene": "UniProtKB:Q9NY33",
  "gene_symbol": "DPP3"
}